{
  "gene": "UniProtKB:O60243",
  "term_id": "GO:0015012",
  "gene_symbol": "HS6ST1",
  "gene_name": "Heparan-sulfate 6-O-sulfotransferase 1",
  "term_label": "heparan sulfate proteoglycan biosynthetic process"
}